{
  "term_label": "mitochondrion organization",
  "gene_name": "Putative coiled-coil-helix-coiled-coil-helix domain-containing protein CHCHD2P9, mitochondrial",
  "term_id": "GO:0007005",
  "gene_symbol": "CHCHD2P9",
  "gene": "UniProtKB:Q5T1J5"
}